{
  "gene": "UniProtKB:Q66K74",
  "gene_name": "Microtubule-associated protein 1S",
  "term_id": "GO:0016358",
  "term_label": "dendrite development",
  "gene_symbol": "MAP1S"
}